{
  "term_label": "homophilic cell-cell adhesion",
  "gene_name": "Carcinoembryonic antigen-related cell adhesion molecule 6",
  "gene_symbol": "CEACAM6",
  "term_id": "GO:0007156",
  "gene": "UniProtKB:P40199"
}